{
  "term_id": "UNKNOWN:0001",
  "gene_name": "Eukaryotic translation initiation factor 3 subunit E",
  "gene": "UniProtKB:P60228",
  "term_label": "Unknown molecular function",
  "gene_symbol": "EIF3E"
}